pressure natriuresis [GO:0003095] (biological process) Subtypes: positive regulation of urine volume by pressure natriuresis [GO:0035818], positive regulation of renal sodium excretion by pressure natriuresis [GO:0035819] Relationships: is a type of renal system process involved in regulation of blood volume [GO:0001977] Definition: The process in which the volume of blood increases renal pressure and thereby results in both an increase in urine volume (diuresis) and an increase in the amount of sodium excreted in the urine (natriuresis). Sources: GOC:mtg_cardio